{
  "term_id": "UNKNOWN:0001",
  "gene_name": "Tubby-related protein 3",
  "term_label": "Unknown molecular function",
  "gene_symbol": "TULP3",
  "gene": "UniProtKB:O75386"
}